renal water absorption [GO:0070295] (biological process) Definition: A renal system process in which water is taken up from the collecting ducts and proximal and distal loops of the nephron. In non-mammalian species, absorption may occur in related structures. Sources: GOC:dph, GOC:mah Also known as: nephron water absorption, renal water reabsorption Relationships: is a type of renal water transport [GO:0003097]; is a type of renal absorption [GO:0070293]